{
  "gene_name": "Thrombospondin type-1 domain-containing protein 7B",
  "gene_symbol": "THSD7B",
  "term_id": "GO:0030036",
  "gene": "UniProtKB:Q9C0I4",
  "term_label": "actin cytoskeleton organization"
}